{
  "gene": "UniProtKB:Q13023",
  "term_id": "GO:0140444",
  "gene_name": "A-kinase anchor protein 6",
  "term_label": "cytoskeleton-nuclear membrane anchor activity",
  "gene_symbol": "AKAP6"
}